{
  "gene_symbol": "EXOC1",
  "gene": "UniProtKB:Q9NV70",
  "term_label": "plasma membrane",
  "term_id": "GO:0005886",
  "gene_name": "Exocyst complex component 1"
}